posterior lateral line neuromast development [GO:0048919] (biological process) Relationships: is_a neuromast development [GO:0048884]; is part of posterior lateral line development [GO:0048916] Sources: ISBN:0125296509 Definition: The process whose specific outcome is the progression of the posterior lateral line neuromast over time, from its formation to the mature structure. The neuromast is the sensory receptor of the anterior lateral line system and is composed of a population of sensory hair cells, and nonsensory supporting cells and mantle cells. Neuromast are located superficially on the epithelium or in lateral line canals.